{
  "gene": "UniProtKB:Q96DC8",
  "term_label": "mitochondrion",
  "gene_symbol": "ECHDC3",
  "gene_name": "Enoyl-CoA hydratase domain-containing protein 3, mitochondrial",
  "term_id": "GO:0005739"
}